{
  "gene": "UniProtKB:Q9HC73",
  "term_label": "receptor complex",
  "gene_name": "Cytokine receptor-like factor 2",
  "term_id": "GO:0043235",
  "gene_symbol": "CRLF2"
}